{
  "term_id": "GO:0010765",
  "gene": "UniProtKB:Q16651",
  "gene_symbol": "PRSS8",
  "gene_name": "Prostasin",
  "term_label": "positive regulation of sodium ion transport"
}